bacterial-type DNA replication initiation [GO:1902328] (biological process) Sources: GOC:TermGenie, GOC:mtg_cell_cycle Also known as: DNA replication initiation involved in bacterial-type DNA replication, DNA-dependent DNA replication initiation involved in bacterial-type DNA replication, DNA endoreduplication initiation involved in bacterial-type DNA replication, DNA re-replication initiation involved in bacterial-type DNA replication Relationships: is a type of cell cycle DNA replication initiation [GO:1902292]; is part of bacterial-type DNA replication [GO:0044787] Definition: Any DNA replication initiation that is involved in bacterial-type DNA replication.